{
  "gene": "UniProtKB:O75131",
  "term_id": "GO:0005544",
  "gene_symbol": "CPNE3",
  "term_label": "calcium-dependent phospholipid binding",
  "gene_name": "Copine-3"
}